{
  "term_id": "GO:0000981",
  "term_label": "DNA-binding transcription factor activity, RNA polymerase II-specific",
  "gene_symbol": "ZNF74",
  "gene_name": "Zinc finger protein 74",
  "gene": "UniProtKB:Q16587"
}